{
  "gene": "UniProtKB:Q9P275",
  "gene_name": "Ubiquitin carboxyl-terminal hydrolase 36",
  "term_id": "GO:0031647",
  "gene_symbol": "USP36",
  "term_label": "regulation of protein stability"
}